{
  "term_id": "GO:0030593",
  "gene_name": "C-X-C chemokine receptor type 2",
  "term_label": "neutrophil chemotaxis",
  "gene": "UniProtKB:P25025",
  "gene_symbol": "CXCR2"
}